gamma-tubulin binding [GO:0043015] (molecular function) Relationships: is a type of GO:0015631 Definition: Binding to the microtubule constituent protein gamma-tubulin. Also known as: gamma tubulin binding Sources: GOC:jl